{
  "term_id": "UNKNOWN:0001",
  "gene_name": "Protein FAM181A",
  "term_label": "Unknown molecular function",
  "gene_symbol": "FAM181A",
  "gene": "UniProtKB:Q8N9Y4"
}